regulation of pentasaccharide transport [GO:1900360] (biological process) Sources: GOC:TermGenie, GOC:mengo_curators Subtypes: regulation of maltopentaose transport [GO:1900315], GO:1900361, positive regulation of pentasaccharide transport [GO:1900362] Definition: Any process that modulates the frequency, rate or extent of pentasaccharide transport. Relationships: is a type of GO:0051049; regulates pentasaccharide transport [GO:2001100]